epithelial cell morphogenesis involved in placental branching [GO:0060672] (biological process) Definition: The change in form (cell shape and size) that occurs when a trophoblast cell elongates to contribute to the branching of the placenta. Relationships: is a type of epithelial cell morphogenesis [GO:0003382]; is a type of embryonic morphogenesis [GO:0048598]; is part of branching involved in labyrinthine layer morphogenesis [GO:0060670]; is part of epithelial cell differentiation involved in embryonic placenta development [GO:0060671] References: PMID:16916377 Sources: GOC:ascb_2009, GOC:dph, GOC:tb